{
  "term_id": "GO:0030182",
  "gene_symbol": "LHX5",
  "gene_name": "LIM_homeobox protein Lhx5",
  "term_label": "neuron differentiation",
  "gene": "UniProtKB:Q9H2C1"
}